{
  "gene": "UniProtKB:Q9NRZ7",
  "term_label": "1-acylglycerol-3-phosphate O-acyltransferase activity",
  "gene_name": "1-acyl-sn-glycerol-3-phosphate acyltransferase gamma",
  "term_id": "GO:0003841",
  "gene_symbol": "AGPAT3"
}